{
  "gene": "UniProtKB:Q5TA81",
  "gene_symbol": "LCE2C",
  "term_label": "Unknown biological process",
  "term_id": "UNKNOWN:0002",
  "gene_name": "Late cornified envelope protein 2C"
}